regulation of DNA metabolic process [GO:0051052] (biological process) Sources: GOC:ai Relationships: is_a regulation of nucleobase-containing compound metabolic process [GO:0019219]; is_a regulation of macromolecule metabolic process [GO:0060255]; regulates DNA metabolic process [GO:0006259] Definition: Any process that modulates the frequency, rate or extent of the chemical reactions and pathways involving DNA. Also known as: regulation of DNA metabolism Subtypes: regulation of DNA recombination [GO:0000018], GO:0006275, regulation of DNA repair [GO:0006282], regulation of telomere maintenance [GO:0032204], negative regulation of DNA metabolic process [GO:0051053], GO:0051054, GO:0060382, regulation of strand invasion [GO:0060542], regulation of DNA strand resection involved in replication fork processing [GO:0110026], regulation of mitochondrial DNA metabolic process [GO:1901858], regulation of mitotic recombination-dependent replication fork processing [GO:1903221], regulation of meiotic DNA double-strand break formation [GO:1903341], regulation of DNA catabolic process [GO:1903624], GO:1903775, GO:2000278